selenocysteine incorporation [GO:0001514] (BP) Sources: RESID:AA0022 Relationships: is a type of GO:0006451 Definition: The incorporation of selenocysteine into a peptide; uses a special tRNA that recognizes the UGA codon as selenocysteine, rather than as a termination codon. Selenocysteine is synthesized from serine before its incorporation; it is not a posttranslational modification of peptidyl-cysteine. Regulation: regulated by regulation of selenocysteine incorporation [GO:1904569]; negatively regulated by negative regulation of selenocysteine incorporation [GO:1904570]; positively regulated by positive regulation of selenocysteine incorporation [GO:1904571]